{
  "gene_name": "Inactive serine_threonine-protein kinase VRK3",
  "term_id": "GO:0005634",
  "gene": "UniProtKB:Q8IV63",
  "gene_symbol": "VRK3",
  "term_label": "nucleus"
}